positive regulation of lysosomal protein catabolic process [GO:1905167] (biological process) Relationships: is a type of positive regulation of protein catabolic process in the vacuole [GO:1904352]; is_a regulation of lysosomal protein catabolic process [GO:1905165]; positively regulates lysosomal protein catabolic process [GO:1905146] Sources: GOC:PARL, GOC:TermGenie, GOC:bf, GO_REF:0000058 Definition: Any process that activates or increases the frequency, rate or extent of lysosomal protein catabolic process. Also known as: positive regulation of cellular protein breakdown in lysosome, positive regulation of cellular protein catabolic process in lysosome, positive regulation of cellular protein catabolism in lysosome, positive regulation of cellular protein degradation in lysosome, positive regulation of lysosomal protein catabolism, positive regulation of lysosomal protein degradation, up regulation of cellular protein breakdown in lysosome, up regulation of cellular protein catabolic process in lysosome, up regulation of cellular protein catabolism in lysosome, up regulation of cellular protein degradation in lysosome, up regulation of lysosomal protein catabolic process, up regulation of lysosomal protein catabolism, up regulation of lysosomal protein degradation, up-regulation of cellular protein breakdown in lysosome, up-regulation of cellular protein catabolic process in lysosome, up-regulation of cellular protein catabolism in lysosome, up-regulation of cellular protein degradation in lysosome, up-regulation of lysosomal protein catabolic process, up-regulation of lysosomal protein catabolism, up-regulation of lysosomal protein degradation, upregulation of cellular protein breakdown in lysosome, upregulation of cellular protein catabolic process in lysosome, upregulation of cellular protein catabolism in lysosome, upregulation of cellular protein degradation in lysosome, upregulation of lysosomal protein catabolic process, upregulation of lysosomal protein catabolism, upregulation of lysosomal protein degradation, activation of cellular protein breakdown in lysosome, activation of cellular protein catabolic process in lysosome, activation of cellular protein catabolism in lysosome, activation of cellular protein degradation in lysosome, activation of lysosomal protein catabolic process, activation of lysosomal protein catabolism, activation of lysosomal protein degradation, activation of lysosomal proteolysis, activation of proteolysis within lysosome, positive regulation of lysosomal proteolysis, positive regulation of proteolysis within lysosome, up regulation of lysosomal proteolysis, up regulation of proteolysis within lysosome, up-regulation of lysosomal proteolysis, up-regulation of proteolysis within lysosome, upregulation of lysosomal proteolysis, upregulation of proteolysis within lysosome